{
  "term_label": "Unknown cellular component",
  "gene": "UniProtKB:Q8TCG1",
  "term_id": "UNKNOWN:0003",
  "gene_name": "Protein CIP2A",
  "gene_symbol": "CIP2A"
}